BAT3 complex [GO:0071818] (cellular component) Relationships: is_a ER membrane insertion complex [GO:0072379] Also known as: BAG6-UBL4A-TRC35 complex, Bag6 complex, BAT3-TRC35-UBL4A complex References: PMID:20676083, PMID:21636303 Sources: GOC:bm Definition: A protein complex found in mammals that transfers tail-anchored (TA) proteins from SGTA to GET3 (ASNA1/TRC4) for targeting to the endoplasmic reticulum membrane. Also chaperones polypeptides from the endoplasmic reticulum retrotranslocation machinery to the proteasome, maintaining the solubility of substrates to improve ER-associated protein degradation (ERAD). Consists of BAG6 (BAT3) and its cofactors GET4 (TRC35) and UBL4A.